positive regulation of synaptic vesicle endocytosis [GO:1900244] (biological process) Relationships: is a type of positive regulation of endocytosis [GO:0045807]; is a type of regulation of synaptic vesicle endocytosis [GO:1900242]; is a type of positive regulation of synaptic vesicle recycling [GO:1903423]; positively regulates synaptic vesicle endocytosis [GO:0048488] Definition: Any process that activates or increases the frequency, rate or extent of synaptic vesicle endocytosis. Also known as: up regulation of synaptic vesicle endocytosis, up-regulation of synaptic vesicle endocytosis, upregulation of synaptic vesicle endocytosis, activation of synaptic vesicle endocytosis, activation of synaptic vesicle retrieval, positive regulation of synaptic vesicle retrieval, up regulation of synaptic vesicle retrieval, up-regulation of synaptic vesicle retrieval, upregulation of synaptic vesicle retrieval Sources: GOC:BHF, GOC:TermGenie